{
  "term_label": "molecular adaptor activity",
  "term_id": "GO:0060090",
  "gene_symbol": "AXIN2",
  "gene": "UniProtKB:Q9Y2T1",
  "gene_name": "Axin-2"
}